activation of bipolar cell growth [GO:0051519] (biological process) Sources: GOC:ai Relationships: is a type of positive regulation of bipolar cell growth [GO:0051518] Definition: Any process that initiates the inactive process of bipolar cell growth, polarized growth from both ends of a cell.